{
  "gene": "UniProtKB:O94923",
  "gene_symbol": "GLCE",
  "term_label": "Golgi apparatus",
  "term_id": "GO:0005794",
  "gene_name": "D-glucuronyl C5-epimerase"
}